{
  "gene_symbol": "NTRK2",
  "gene_name": "BDNF_NT-3 growth factors receptor",
  "term_label": "receptor complex",
  "gene": "UniProtKB:Q16620",
  "term_id": "GO:0043235"
}